{
  "term_label": "Unknown molecular function",
  "gene_symbol": "TMSB15C",
  "term_id": "UNKNOWN:0001",
  "gene_name": "Thymosin beta-15C",
  "gene": "UniProtKB:P0DX04"
}